{
  "term_label": "mitochondrial matrix",
  "term_id": "GO:0005759",
  "gene_name": "Lon protease homolog, mitochondrial",
  "gene_symbol": "LONP1",
  "gene": "UniProtKB:P36776"
}